{
  "gene": "UniProtKB:D6R9N7",
  "term_label": "cysteine-type deubiquitinase activity",
  "gene_name": "Ubiquitin carboxyl-terminal hydrolase 17-like protein 18",
  "term_id": "GO:0004843",
  "gene_symbol": "USP17L18"
}